positive regulation of signal transduction by p53 class mediator [GO:1901798] (biological process) Definition: Any process that activates or increases the frequency, rate or extent of signal transduction by p53 class mediator. Relationships: is_a regulation of signal transduction by p53 class mediator [GO:1901796]; is_a GO:1902533; positively regulates GO:0072331 Subtypes: positive regulation of DNA damage response, signal transduction by p53 class mediator [GO:0043517], positive regulation of intrinsic apoptotic signaling pathway by p53 class mediator [GO:1902255] Also known as: up regulation of signal transduction by p53 class mediator, up-regulation of signal transduction by p53 class mediator, upregulation of signal transduction by p53 class mediator, activation of signal transduction by p53 class mediator Sources: GOC:TermGenie